{
  "term_label": "signaling receptor activator activity",
  "gene": "UniProtKB:P05067",
  "term_id": "GO:0030546",
  "gene_symbol": "APP",
  "gene_name": "Amyloid-beta precursor protein"
}